positive regulation of potassium ion transmembrane transport [GO:1901381] (BP) Definition: Any process that activates or increases the frequency, rate or extent of potassium ion transmembrane transport. Also known as: positive regulation of potassium ion membrane transport, up regulation of potassium ion transmembrane transport, up-regulation of potassium ion transmembrane transport, upregulation of potassium ion transmembrane transport, activation of potassium ion transmembrane transport Relationships: is a type of positive regulation of potassium ion transport [GO:0043268]; is_a regulation of potassium ion transmembrane transport [GO:1901379]; is a type of GO:1904064; positively regulates potassium ion transmembrane transport [GO:0071805] Sources: GOC:BHF, GOC:TermGenie Subtypes: positive regulation of potassium ion import across plasma membrane [GO:1903288], positive regulation of potassium ion export across plasma membrane [GO:1903766]